positive regulation of cell activation [GO:0050867] (biological process) Also known as: up regulation of cell activation, up-regulation of cell activation, upregulation of cell activation, activation of cell activation, stimulation of cell activation Relationships: is a type of positive regulation of cellular process [GO:0048522]; is_a GO:0050865; is a type of GO:0051240; positively regulates cell activation [GO:0001775] Sources: GOC:ai Subtypes: GO:0002696, GO:0010572, GO:0014718, positive regulation of astrocyte activation [GO:0061890], positive regulation of endothelial cell activation [GO:1904989], positive regulation of hepatic stellate cell activation [GO:2000491] Definition: Any process that activates or increases the frequency, rate or extent of activation.